{
  "gene_symbol": "CHRNA5",
  "gene": "UniProtKB:P30532",
  "gene_name": "Neuronal acetylcholine receptor subunit alpha-5",
  "term_id": "GO:0007274",
  "term_label": "neuromuscular synaptic transmission"
}